positive regulation of seed maturation [GO:2000693] (biological process) Definition: Any process that activates or increases the frequency, rate or extent of seed maturation. Sources: GOC:obol Relationships: is a type of positive regulation of developmental process [GO:0051094]; is a type of positive regulation of multicellular organismal process [GO:0051240]; is a type of regulation of seed maturation [GO:2000034]; is a type of positive regulation of reproductive process [GO:2000243]; positively regulates seed maturation [GO:0010431]